{
  "gene_symbol": "PEX26",
  "gene_name": "Peroxisome assembly protein 26",
  "gene": "UniProtKB:Q7Z412",
  "term_id": "GO:0016558",
  "term_label": "protein import into peroxisome matrix"
}